urate biosynthetic process [GO:0034418] (biological process) Definition: The chemical reactions and pathways resulting in the formation of urate, the anion of uric acid, 2,6,8-trioxypurine. Sources: GOC:mah Relationships: is a type of GO:0044283; is a type of urate metabolic process [GO:0046415]; is a type of purine-containing compound biosynthetic process [GO:0072522] Also known as: urate biosynthesis, urate formation, urate synthesis, uric acid biosynthetic process, urate anabolism